{
  "term_id": "UNKNOWN:0003",
  "term_label": "Unknown cellular component",
  "gene_symbol": "PLAC1",
  "gene": "UniProtKB:Q9HBJ0",
  "gene_name": "Placenta-specific protein 1"
}